{
  "term_id": "UNKNOWN:0001",
  "gene_name": "Lymphocyte antigen 6 complex locus protein G6f",
  "gene_symbol": "LY6G6F",
  "gene": "UniProtKB:Q5SQ64",
  "term_label": "Unknown molecular function"
}